regulation of phosphatase activity [GO:0010921] (biological process) Sources: GOC:BHF, GOC:dph, GOC:tb Subtypes: positive regulation of phosphatase activity [GO:0010922], negative regulation of phosphatase activity [GO:0010923] Relationships: is a type of GO:0035303; is a type of regulation of hydrolase activity [GO:0051336]; regulates phosphatase activity [GO:0016791] Definition: Any process that modulates the rate or frequency of phosphatase activity. Phosphatases catalyze the hydrolysis of phosphoric monoesters, releasing phosphate.